paracellular tight junction channel activity [GO:0160187] (molecular function) Also known as: claudin pore Definition: Enables size- and charge-selective transport of solutes through a tight junction barrier paracellularly, across the epithelium. References: PMID:30665499 Relationships: is a type of transporter activity [GO:0005215]